{
  "gene_symbol": "AK4P3",
  "gene_name": "Adenylate kinase 4, mitochondrial",
  "term_label": "nucleoside diphosphate kinase activity",
  "term_id": "GO:0004550",
  "gene": "UniProtKB:A0A8I5KW96"
}